{
  "gene_name": "GRAM domain-containing protein 2B",
  "gene_symbol": "GRAMD2B",
  "term_label": "Unknown molecular function",
  "gene": "UniProtKB:Q96HH9",
  "term_id": "UNKNOWN:0001"
}